{
  "gene": "UniProtKB:Q6IE37",
  "gene_name": "Ovostatin homolog 1",
  "term_id": "UNKNOWN:0003",
  "term_label": "Unknown cellular component",
  "gene_symbol": "OVOS1"
}